{
  "gene_symbol": "ABCB5",
  "term_id": "GO:0042626",
  "gene": "UniProtKB:Q2M3G0",
  "gene_name": "ATP-binding cassette sub-family B member 5",
  "term_label": "ATPase-coupled transmembrane transporter activity"
}